{
  "gene_name": "CD209 antigen",
  "term_label": "D-mannose binding",
  "term_id": "GO:0005537",
  "gene_symbol": "CD209",
  "gene": "UniProtKB:Q9NNX6"
}